transmembrane histidine kinase cytokinin receptor activity [GO:0009885] (molecular function) Sources: GOC:lr, GOC:mah Definition: Combining with a cytokinin and transmitting the signal from one side of the membrane to the other to initiate a change in cell activity by catalysis of the reaction: ATP + a protein-L-histidine = ADP + a protein-L-histidine phosphate. Relationships: is a type of transmembrane receptor histidine kinase activity [GO:0009784]; is a type of cytokinin receptor activity [GO:0009884]